{
  "gene": "UniProtKB:Q8WXH4",
  "term_label": "positive regulation of protein catabolic process",
  "gene_name": "Ankyrin repeat and SOCS box protein 11",
  "gene_symbol": "ASB11",
  "term_id": "GO:0045732"
}